{
  "gene_name": "Extracellular matrix organizing protein FRAS1",
  "gene_symbol": "FRAS1",
  "term_label": "cell-matrix adhesion",
  "gene": "UniProtKB:Q86XX4",
  "term_id": "GO:0007160"
}